positive regulation of lactation [GO:1903489] (biological process) Definition: Any process that activates or increases the frequency, rate or extent of lactation. References: PMID:19563620 Sources: GOC:TermGenie, GOC:mr, GO_REF:0000058 Also known as: up regulation of lactation, up-regulation of lactation, upregulation of lactation, activation of lactation Relationships: is a type of positive regulation of secretion [GO:0051047]; is a type of positive regulation of developmental process [GO:0051094]; is a type of positive regulation of multicellular organismal process [GO:0051240]; is a type of GO:1903487; positively regulates GO:0007595 Subtypes: positive regulation of lactation by mesenchymal-epithelial cell signaling [GO:0060637]